{
  "term_id": "GO:0061133",
  "gene": "UniProtKB:Q9UL46",
  "gene_name": "Proteasome activator complex subunit 2",
  "term_label": "endopeptidase activator activity",
  "gene_symbol": "PSME2"
}